{
  "gene_name": "Insulin receptor",
  "gene": "UniProtKB:P06213",
  "term_id": "GO:0051897",
  "term_label": "positive regulation of phosphatidylinositol 3-kinase/protein kinase B signal transduction",
  "gene_symbol": "INSR"
}